{
  "gene": "UniProtKB:Q8N7Q2",
  "gene_symbol": "CELF2-AS1",
  "gene_name": "Putative uncharacterized protein CELF2-AS1",
  "term_label": "Unknown cellular component",
  "term_id": "UNKNOWN:0003"
}